beta-ketoadipate pathway [GO:0042952] (biological process) Subtypes: GO:0019615 References: PMID:8905091 Sources: GOC:jl Relationships: is_a GO:0009056 Also known as: ortho-cleavage pathway Definition: A pathway of aromatic compound degradation by ortho-cleavage; one branch converts protocatechuate, derived from phenolic compounds, to beta-ketoadipate, and the other branch converts catechol, generated from various aromatic hydrocarbons, amino aromatics, and lignin monomers, also to beta-ketoadipate. Two additional steps accomplish the conversion of beta-ketoadipate to tricarboxylic acid cycle intermediates.